{
  "gene": "UniProtKB:Q15699",
  "gene_name": "ALX homeobox protein 1",
  "gene_symbol": "ALX1",
  "term_label": "negative regulation of DNA-templated transcription",
  "term_id": "GO:0045892"
}